mammary gland development [GO:0030879] (biological process) References: PMID:9576833 Relationships: is a type of GO:0048732 Also known as: mammogenesis Definition: The process whose specific outcome is the progression of the mammary gland over time, from its formation to the mature structure. The mammary gland is a large compound sebaceous gland that in female mammals is modified to secrete milk. Its development starts with the formation of the mammary line and ends as the mature gland cycles between nursing and weaning stages.